{
  "gene_name": "Cytokine receptor-like factor 1",
  "gene": "UniProtKB:O75462",
  "term_id": "GO:0043524",
  "term_label": "negative regulation of neuron apoptotic process",
  "gene_symbol": "CRLF1"
}